{
  "term_id": "GO:0030425",
  "gene_symbol": "HOMER3",
  "term_label": "dendrite",
  "gene_name": "Homer protein homolog 3",
  "gene": "UniProtKB:Q9NSC5"
}